{
  "term_id": "GO:0007186",
  "term_label": "G protein-coupled receptor signaling pathway",
  "gene_symbol": "GPR52",
  "gene_name": "G-protein coupled receptor 52",
  "gene": "UniProtKB:Q9Y2T5"
}